polo box domain specific binding [GO:0090488] (molecular function) Definition: Binding to a polo box domain of a protein. The polo box domain is involved in binding substrates of polo kinases. References: PMID:12352953 Sources: GOC:al, GOC:tb, Pfam:PF00659 Relationships: is a type of GO:0019904